{
  "gene_name": "Ribosomal protein S6 kinase alpha-2",
  "gene": "UniProtKB:Q15349",
  "term_id": "GO:0005737",
  "gene_symbol": "RPS6KA2",
  "term_label": "cytoplasm"
}